{
  "term_id": "GO:0005886",
  "gene_name": "Ephrin-B2",
  "term_label": "plasma membrane",
  "gene": "UniProtKB:P52799",
  "gene_symbol": "EFNB2"
}